{
  "gene_name": "Integrin-linked protein kinase",
  "term_id": "GO:0005737",
  "term_label": "cytoplasm",
  "gene": "UniProtKB:Q13418",
  "gene_symbol": "ILK"
}